lithocholic acid binding [GO:1902121] (molecular function) References: PMID:20371703 Sources: GOC:TermGenie, GOC:bf Definition: Binding to lithocholic acid. Relationships: is a type of steroid binding [GO:0005496]; is a type of bile acid binding [GO:0032052] Also known as: LCA binding